{
  "gene_symbol": "ARHGEF18",
  "term_label": "plasma membrane",
  "term_id": "GO:0005886",
  "gene_name": "Rho guanine nucleotide exchange factor 18 (Fragment)",
  "gene": "UniProtKB:A0A590UK10"
}